{
  "term_id": "GO:0000978",
  "term_label": "RNA polymerase II cis-regulatory region sequence-specific DNA binding",
  "gene_symbol": "ZNF714",
  "gene_name": "Zinc finger protein 714",
  "gene": "UniProtKB:Q96N38"
}